linear element [GO:0030998] (cellular component) Relationships: is a type of synaptonemal structure [GO:0099086] References: PMID:12665553, PMID:30640914 Sources: DOI:10.2323/jgam.28.263, GOC:jb Definition: A proteinaceous scaffold associated with fission yeast chromosomes during meiotic prophase. Linear elements consist of a protein complex, LinE, with four main structural components (Rec10, Rec25, Rec27, and Mug20 in S. pombe) associated with chromatin. The resulting structure is related to but not equivalent to the synaptonemal complex.